{
  "gene_symbol": "TRUB1",
  "term_label": "nucleus",
  "gene": "UniProtKB:Q8WWH5",
  "term_id": "GO:0005634",
  "gene_name": "Pseudouridylate synthase TRUB1"
}